{
  "gene_symbol": "PMS2P3",
  "term_id": "UNKNOWN:0003",
  "term_label": "Unknown cellular component",
  "gene_name": "Putative postmeiotic segregation increased 2-like protein 3",
  "gene": "UniProtKB:Q13401"
}